{
  "term_id": "GO:0005886",
  "gene_name": "Synembryn-A",
  "term_label": "plasma membrane",
  "gene_symbol": "RIC8A",
  "gene": "UniProtKB:Q9NPQ8"
}